hydroxyisourate hydrolase complex [GO:0106232] (cellular component) Definition: A hydrolase complex that converts 5-hydroxyisourate (HIU) to 2-oxo-4-hydroxy-4-carboxy-5-ureidoimidazoline. This is the second step of the three-step enzymatic reaction that degrades uric acid to (S)-allantoin. References: PMID:21795808 Sources: GOC:bhm Also known as: 5-hydroxyisourate hydrolase complex, HIU hydrolase complex, HIUH complex Relationships: is a type of catalytic complex [GO:1902494]; is part of GO:0005737